{
  "gene_symbol": "SMYD2",
  "gene": "UniProtKB:Q9NRG4",
  "term_id": "GO:0045892",
  "gene_name": "N-lysine methyltransferase SMYD2",
  "term_label": "negative regulation of DNA-templated transcription"
}